plant organ senescence [GO:0090693] (biological process) Subtypes: leaf senescence [GO:0010150], GO:0080187 Definition: A plant organ developmental process during which a plant dismantles cellular components to reclaim the cellular building blocks and nutrients that have been deposited in the plant organs during growth. References: PMID:17177638, PMID:34938309 Sources: GOC:tb Relationships: is_a developmental process [GO:0032502]; is part of plant organ development [GO:0099402]